{
  "gene_name": "Zinc finger protein 800",
  "term_id": "UNKNOWN:0001",
  "term_label": "Unknown molecular function",
  "gene": "UniProtKB:Q2TB10",
  "gene_symbol": "ZNF800"
}